{
  "gene_name": "Olfactory receptor 4N2",
  "gene_symbol": "OR4N2",
  "gene": "UniProtKB:Q8NGD1",
  "term_id": "GO:0005886",
  "term_label": "plasma membrane"
}